{
  "gene": "UniProtKB:Q86VG3",
  "gene_name": "Intraflagellar transport-associated protein",
  "term_id": "GO:0120160",
  "term_label": "intraciliary transport particle A binding",
  "gene_symbol": "IFTAP"
}